{
  "gene_name": "Tubulin beta-4A chain",
  "gene": "UniProtKB:P04350",
  "term_id": "GO:0005200",
  "gene_symbol": "TUBB4A",
  "term_label": "structural constituent of cytoskeleton"
}